GTPase activator complex [GO:1902773] (cellular component) Note: An example of this is BFA1 in Saccharomyces cerevisiae (P47113) in PMID:16449187 (inferred from direct assay). References: PMID:16449187 Sources: GOC:TermGenie, GOC:bhm, GO_REF:0000088 Definition: A protein complex which is capable of GTPase activator activity. Subtypes: Bfa1-Bub2 complex [GO:1990334], FNIP-folliculin RagC/D GAP [GO:1990877] Relationships: is a type of GO:0150005